{
  "gene_name": "Peroxisomal multifunctional enzyme type 2",
  "term_label": "(3R)-3-hydroxyacyl-CoA dehydrogenase (NAD+) activity",
  "gene": "UniProtKB:P51659",
  "term_id": "GO:0106386",
  "gene_symbol": "HSD17B4"
}